{
  "gene": "UniProtKB:Q13542",
  "gene_symbol": "EIF4EBP2",
  "term_label": "eukaryotic initiation factor 4E binding",
  "gene_name": "Eukaryotic translation initiation factor 4E-binding protein 2",
  "term_id": "GO:0008190"
}